{
  "term_id": "GO:0005125",
  "gene_symbol": "GDF9",
  "term_label": "cytokine activity",
  "gene_name": "Growth_differentiation factor 9",
  "gene": "UniProtKB:O60383"
}